{
  "gene": "UniProtKB:Q6UX73",
  "term_id": "UNKNOWN:0001",
  "gene_name": "UPF0764 protein C16orf89",
  "term_label": "Unknown molecular function",
  "gene_symbol": "C16orf89"
}